{
  "gene_name": "Homeobox protein engrailed-2",
  "gene_symbol": "EN2",
  "term_id": "GO:0006357",
  "gene": "UniProtKB:P19622",
  "term_label": "regulation of transcription by RNA polymerase II"
}